{
  "gene_name": "Spindle and kinetochore-associated protein 3",
  "gene_symbol": "SKA3",
  "term_id": "GO:0007059",
  "term_label": "chromosome segregation",
  "gene": "UniProtKB:Q8IX90"
}